{
  "gene_name": "Uncharacterized protein",
  "gene_symbol": "Q6YL49",
  "gene": "UniProtKB:Q6YL49",
  "term_label": "Unknown biological process",
  "term_id": "UNKNOWN:0002"
}